{
  "term_id": "UNKNOWN:0003",
  "term_label": "Unknown cellular component",
  "gene": "UniProtKB:Q02325",
  "gene_symbol": "PLGLB2",
  "gene_name": "Plasminogen-like protein B"
}